{
  "term_label": "extracellular space",
  "term_id": "GO:0005615",
  "gene": "UniProtKB:Q5T4W7",
  "gene_symbol": "ARTN",
  "gene_name": "Artemin"
}